UDP-4-amino-4-deoxy-L-arabinose aminotransferase [GO:0099620] (molecular function) Also known as: UDP-(beta-L-threo-pentapyranosyl-4''-ulose diphosphate) aminotransferase, UDP-4-amino-4-deoxy-L-arabinose---oxoglutarate aminotransferase, UDP-4-amino-4-deoxy-beta-L-arabinose:2-oxoglutarate aminotransferase, UDP-Ara4O aminotransferase, UDP-L-Ara4N transaminase References: PMID:12429098, PMID:12704196 Sources: GOC:al, GOC:dos Relationships: is a type of transaminase activity [GO:0008483] Definition: Catalysis of the reaction: UDP-4-amino-4-deoxy-beta-L-arabinopyranose + 2-oxoglutarate = UDP-beta-L-threo-pentapyranos-4-ulose + L-glutamate.